positive regulation of transcription of Notch receptor target [GO:0007221] (BP) Definition: The activation of transcription of specific genes as a result of Notch signaling, mediated by the Notch intracellular domain. Also known as: N receptor target transcription factor activation, Notch receptor target transcription factor activation References: PMID:12651094 Relationships: is a type of positive regulation of transcription by RNA polymerase II [GO:0045944]; is part of Notch signaling pathway [GO:0007219]